adhesion of symbiont to host cell [GO:0044650] (biological process) Definition: The attachment of a symbiont to a host cell via adhesion molecules, general stickiness etc., either directly or indirectly. Sources: GOC:jl Relationships: is a type of GO:0044406 Subtypes: virion attachment to host cell [GO:0019062], adhesion of symbiont to microvasculature [GO:0020035], adhesion of symbiont to host epithelial cell [GO:0044651], GO:0044652, adhesion to host cell via type IV pili [GO:0052001], adhesion of symbiont spore to host [GO:0075004], adhesion of symbiont to host cell surface via host membrane carbohydrate [GO:0141024], GO:0141025, GO:0141026